endoplasmic reticulum disassembly [GO:1905692] (biological process) Relationships: is a type of GO:0007029; is a type of organelle disassembly [GO:1903008] Also known as: ER disassembly Definition: The disaggregation of an endoplasmic reticulum into its constituent components. Sources: GOC:TermGenie, GOC:autophagy, GOC:pr, GO_REF:0000079